{
  "gene": "UniProtKB:Q6ZRF8",
  "term_label": "regulation of cardiac muscle contraction",
  "gene_name": "RING finger protein 207",
  "gene_symbol": "RNF207",
  "term_id": "GO:0055117"
}